{
  "term_label": "Unknown cellular component",
  "term_id": "UNKNOWN:0003",
  "gene_name": "Sperm-egg fusion protein LLCFC1",
  "gene_symbol": "LLCFC1",
  "gene": "UniProtKB:Q96L11"
}